alcohol O-cinnamoyltransferase activity [GO:0047182] (molecular function) Definition: Catalysis of the reaction: an alcohol + 1-O-trans-cinnamoyl-beta-D-glucopyranose = beta-D-glucose + alkyl cinnamate. Sources: EC:2.3.1.152, MetaCyc:2.3.1.152-RXN Also known as: 1-O-trans-cinnamoyl-beta-D-glucopyranose:alcohol O-cinnamoyltransferase activity Relationships: is a type of acyltransferase activity, transferring groups other than amino-acyl groups [GO:0016747]